{
  "term_id": "UNKNOWN:0002",
  "gene": "UniProtKB:Q9HCN8",
  "gene_name": "Stromal cell-derived factor 2-like protein 1",
  "term_label": "Unknown biological process",
  "gene_symbol": "SDF2L1"
}